{
  "gene_name": "Lysozyme C",
  "term_id": "GO:0050829",
  "gene": "UniProtKB:P61626",
  "term_label": "defense response to Gram-negative bacterium",
  "gene_symbol": "LYZ"
}